L-methionine catabolic process to succinyl-CoA [GO:0019457] (BP) Sources: GOC:go_curators Relationships: is a type of GO:0006104; is a type of L-methionine catabolic process [GO:0009087]; is a type of amide catabolic process [GO:0043605] Also known as: methionine breakdown to succinyl-CoA, methionine degradation to succinyl-CoA Definition: The chemical reactions and pathways resulting in the breakdown of L-methionine into other compounds, including succinyl-CoA.